{
  "term_id": "UNKNOWN:0003",
  "gene_symbol": "TRAV1-2",
  "gene_name": "T cell receptor alpha variable 1-2",
  "gene": "UniProtKB:A0A0B4J238",
  "term_label": "Unknown cellular component"
}